{
  "gene_symbol": "PKP1",
  "term_label": "adherens junction",
  "term_id": "GO:0005912",
  "gene_name": "Plakophilin-1",
  "gene": "UniProtKB:Q13835"
}